{
  "gene_symbol": "FGF17",
  "gene_name": "Fibroblast growth factor 17",
  "term_label": "cytoplasm",
  "term_id": "GO:0005737",
  "gene": "UniProtKB:O60258"
}